histone H2B kinase activity [GO:0140998] (molecular function) References: PMID:25303536 Relationships: is a type of histone kinase activity [GO:0035173] Subtypes: histone H2BS14 kinase activity [GO:0044025], histone H2BS36 kinase activity [GO:0140823] Definition: Catalysis of the transfer of a phosphate group to a histone H2B.